{
  "term_label": "cytoplasmic translation",
  "gene_symbol": "RPS29",
  "gene_name": "Small ribosomal subunit protein uS14",
  "term_id": "GO:0002181",
  "gene": "UniProtKB:P62273"
}